deacetylisoipecoside synthase activity [GO:0050556] (molecular function) Definition: Catalysis of the reaction: deacetylisoipecoside + H2O = dopamine + secologanin. Also known as: deacetylisoipecoside dopamine-lyase (secologanin-forming), deacetylisoipecoside dopamine-lyase activity Relationships: is a type of hydrolase activity, acting on carbon-nitrogen (but not peptide) bonds [GO:0016810] Sources: RHEA:21756